{
  "gene": "UniProtKB:Q9NVA2",
  "gene_name": "Septin-11",
  "term_label": "cytoskeleton-dependent cytokinesis",
  "gene_symbol": "SEPTIN11",
  "term_id": "GO:0061640"
}